{
  "gene_name": "Protein mono-ADP-ribosyltransferase TIPARP",
  "gene": "UniProtKB:Q7Z3E1",
  "term_id": "GO:0005634",
  "gene_symbol": "TIPARP",
  "term_label": "nucleus"
}